{
  "gene": "UniProtKB:Q9BU70",
  "term_id": "GO:0089715",
  "gene_name": "tRNA (adenine(37)-N6)-methyltransferase",
  "term_label": "tRNA (L-threonylcarbamoyladenosine(37)-C2) methyltransferase activity",
  "gene_symbol": "TRMO"
}